GPI mannosyltransferase activity [GO:0004376] (MF) Also known as: glycolipid mannosyltransferase activity, glycolipid mannosyl transferase activity Definition: Catalysis of the transfer of an alpha-D-mannosyl residue from dolichol-P-mannose to GlcN-acyl-PI bearing 0-3 mannoses during formation of the GPI precursor. Relationships: is a type of mannosyltransferase activity [GO:0000030] Subtypes: dol-P-Man:Man(1)GlcN-acyl-PI alpha-1,6-mannosyltransferase activity [GO:0120563], GO:0120564, dol-P-Man:Man(3)GlcN-acyl-PI alpha-1,2-mannosyltransferase activity [GO:0120565], GO:0180041 Sources: GOC:curators